{
  "term_label": "cytoplasm",
  "gene_name": "Inactive serine_threonine-protein kinase VRK3",
  "term_id": "GO:0005737",
  "gene_symbol": "VRK3",
  "gene": "UniProtKB:Q8IV63"
}